negative regulation of iron-sulfur cluster assembly [GO:1903330] (biological process) Relationships: is a type of GO:0051129; is a type of regulation of iron-sulfur cluster assembly [GO:1903329]; negatively regulates GO:0016226 Definition: Any process that stops, prevents or reduces the frequency, rate or extent of iron-sulfur cluster assembly. Subtypes: GO:1900488, negative regulation of [4Fe-4S] cluster assembly [GO:1900492], negative regulation of iron-sulfur-molybdenum cofactor assembly [GO:1900507] Also known as: down regulation of iron-sulfur cluster assembly, down regulation of iron-sulphur cluster assembly, down-regulation of iron-sulfur cluster assembly, down-regulation of iron-sulphur cluster assembly, downregulation of iron-sulfur cluster assembly, downregulation of iron-sulphur cluster assembly, negative regulation of iron-sulphur cluster assembly, inhibition of iron-sulfur cluster assembly, inhibition of iron-sulphur cluster assembly, down regulation of iron-sulfur cluster biosynthesis, down-regulation of iron-sulfur cluster biosynthesis, downregulation of iron-sulfur cluster biosynthesis, inhibition of iron-sulfur cluster biosynthesis, negative regulation of iron-sulfur cluster biosynthesis Sources: GOC:TermGenie, GOC:vw, GO_REF:0000058